neutrophil degranulation [GO:0043312] (biological process) Definition: The regulated exocytosis of secretory granules containing preformed mediators such as proteases, lipases, and inflammatory mediators by a neutrophil. Sources: ISBN:0781735149 Also known as: neutrophil granule exocytosis, heterophil degranulation Relationships: is a type of GO:0043299; is part of GO:0002283; is part of neutrophil mediated immunity [GO:0002446] Regulation: regulated by regulation of neutrophil degranulation [GO:0043313]; negatively regulated by negative regulation of neutrophil degranulation [GO:0043314]; positively regulated by positive regulation of neutrophil degranulation [GO:0043315]